{
  "gene_name": "Gamma-aminobutyric acid receptor-associated protein",
  "term_id": "GO:0006995",
  "term_label": "cellular response to nitrogen starvation",
  "gene": "UniProtKB:O95166",
  "gene_symbol": "GABARAP"
}